{
  "gene": "UniProtKB:Q9UK45",
  "gene_symbol": "LSM7",
  "term_label": "Unknown biological process",
  "term_id": "UNKNOWN:0002",
  "gene_name": "U6 snRNA-associated Sm-like protein LSm7"
}